G-protein beta/gamma-Btk complex [GO:0070441] (cellular component) Definition: A protein complex formed by the association of the Bruton tyrosine protein kinase Btk, which is implicated in mammalian X-linked immunodeficiencies, with the beta and gamma subunits of a heterotrimeric G protein. Also known as: G protein complex (BTK, GNG1, GNG2), G protein complex (Btk, Gng2, Gnb1) Relationships: is a type of protein-containing complex [GO:0032991]; is part of cytoplasm [GO:0005737] References: PMID:7972043 Sources: GOC:mah Note: See also the cellular component term 'heterotrimeric G-protein complex ; GO:0005834'.